{
  "term_id": "UNKNOWN:0003",
  "gene_symbol": "CRYGB",
  "term_label": "Unknown cellular component",
  "gene": "UniProtKB:P07316",
  "gene_name": "Gamma-crystallin B"
}